{
  "gene_name": "Centrosomal protein of 19 kDa",
  "gene_symbol": "CEP19",
  "term_id": "GO:0005813",
  "term_label": "centrosome",
  "gene": "UniProtKB:Q96LK0"
}